farnesoate epoxidase activity [GO:0120512] (molecular function) Relationships: is a type of GO:0016712 Definition: Catalysis of the reaction: (2E,6E)-farnesoate + O2 + reduced [NADPH--hemoprotein reductase] = H+ + H2O + juvenile hormone III carboxylate + oxidized [NADPH--hemoprotein reductase]. Also known as: CYP15C1 activity References: PMID:22412378, PMID:38741075 Sources: RHEA:43724